{
  "gene_symbol": "FAM83B",
  "term_id": "GO:0005737",
  "term_label": "cytoplasm",
  "gene": "UniProtKB:Q5T0W9",
  "gene_name": "Protein FAM83B"
}